extrinsic component of thylakoid membrane [GO:0035448] (cellular component) Sources: GOC:bf, GOC:dos Definition: The component of a thylakoid membrane consisting of gene products and protein complexes that are loosely bound to one of its surfaces, but not integrated into the hydrophobic region. Subtypes: extrinsic component of plastid thylakoid membrane [GO:0035449] Relationships: is_a extrinsic component of membrane [GO:0019898]; is part of GO:0042651 Also known as: peripheral to thylakoid membrane, extrinsic to thylakoid membrane